peregrinol diphosphate synthase activity [GO:0106238] (molecular function) Definition: Catalysis of the reaction:peregrinol diphosphate = all-trans-geranylgeranyl diphosphate + H2O. References: PMID:24990389, PMID:29315936 Sources: GOC:emb, RHEA:54652 Relationships: is a type of GO:0016836